imaginal disc-derived leg joint morphogenesis [GO:0016348] (biological process) Relationships: is a type of post-embryonic animal morphogenesis [GO:0009886]; is part of GO:0036011 Definition: The process in which the anatomical structures of an imaginal disc-derived leg joint are generated and organized. The leg joint is a flexible region that separates the rigid sections of a leg to allow movement in a controlled manner. An example of this is found in Drosophila melanogaster. Sources: GOC:mtg_sensu, ISBN:0879694238